{
  "term_id": "GO:0003723",
  "gene_symbol": "RPS4Y1",
  "gene_name": "Small ribosomal subunit protein eS4, Y isoform 1",
  "gene": "UniProtKB:P22090",
  "term_label": "RNA binding"
}